{
  "gene_symbol": "EIF1",
  "term_id": "GO:0043024",
  "gene_name": "Eukaryotic translation initiation factor 1",
  "term_label": "ribosomal small subunit binding",
  "gene": "UniProtKB:P41567"
}